{
  "gene": "UniProtKB:O95817",
  "gene_symbol": "BAG3",
  "term_label": "muscle cell cellular homeostasis",
  "term_id": "GO:0046716",
  "gene_name": "BAG family molecular chaperone regulator 3"
}